{
  "gene": "UniProtKB:A1L3X4",
  "gene_symbol": "MT1DP",
  "term_id": "GO:0071294",
  "term_label": "cellular response to zinc ion",
  "gene_name": "Putative metallothionein MT1DP"
}